{
  "gene": "UniProtKB:Q9UI25",
  "term_id": "UNKNOWN:0002",
  "gene_name": "Putative uncharacterized protein PRO0461",
  "term_label": "Unknown biological process",
  "gene_symbol": "PRO0461"
}